positive regulation of tubulin deacetylation [GO:0090044] (biological process) Sources: GOC:BHF, GOC:dph, GOC:tb Definition: Any process that increases the frequency, rate or extent of tubulin deacetylation. Tubulin deacetylation is the removal of an acetyl group from a protein amino acid. Relationships: is a type of regulation of tubulin deacetylation [GO:0090043]; is a type of positive regulation of protein deacetylation [GO:0090312]; positively regulates tubulin deacetylation [GO:0090042]